positive regulation of slow-twitch skeletal muscle fiber contraction [GO:0031451] (biological process) Also known as: positive regulation of slow-twitch skeletal muscle contraction, up regulation of slow-twitch skeletal muscle contraction, up-regulation of slow-twitch skeletal muscle contraction, upregulation of slow-twitch skeletal muscle contraction, activation of slow-twitch skeletal muscle contraction, stimulation of slow-twitch skeletal muscle contraction Sources: GOC:dph, GOC:ef, GOC:mah, GOC:mtg_muscle, GOC:tb Relationships: is a type of regulation of slow-twitch skeletal muscle fiber contraction [GO:0031449]; is a type of positive regulation of striated muscle contraction [GO:0045989]; positively regulates GO:0031444 Definition: Any process that activates or increases the frequency, rate or extent of slow-twitch skeletal muscle contraction.